{
  "term_id": "GO:0005634",
  "gene_name": "Calcium_calmodulin-dependent protein kinase type IV",
  "gene": "UniProtKB:Q16566",
  "term_label": "nucleus",
  "gene_symbol": "CAMK4"
}